{
  "gene_name": "Activin receptor type-1C",
  "gene_symbol": "ACVR1C",
  "term_id": "GO:0032924",
  "term_label": "activin receptor signaling pathway",
  "gene": "UniProtKB:Q8NER5"
}